{
  "term_label": "cytoplasm",
  "gene_name": "Serine_threonine-protein kinase DCLK1",
  "term_id": "GO:0005737",
  "gene": "UniProtKB:O15075",
  "gene_symbol": "DCLK1"
}